{
  "gene": "UniProtKB:Q9H239",
  "term_id": "GO:0030198",
  "term_label": "extracellular matrix organization",
  "gene_name": "Matrix metalloproteinase-28",
  "gene_symbol": "MMP28"
}